{
  "gene": "UniProtKB:Q99811",
  "term_label": "RNA polymerase II cis-regulatory region sequence-specific DNA binding",
  "gene_symbol": "PRRX2",
  "gene_name": "Paired mesoderm homeobox protein 2",
  "term_id": "GO:0000978"
}